{
  "term_label": "RNA polymerase II cis-regulatory region sequence-specific DNA binding",
  "term_id": "GO:0000978",
  "gene_name": "B-cell lymphoma_leukemia 11B",
  "gene_symbol": "BCL11B",
  "gene": "UniProtKB:Q9C0K0"
}